{
  "term_id": "UNKNOWN:0003",
  "gene_name": "FXYD domain-containing ion transport regulator 6",
  "gene": "UniProtKB:Q9H0Q3",
  "term_label": "Unknown cellular component",
  "gene_symbol": "FXYD6"
}